lipid droplet organization [GO:0034389] (biological process) References: PMID:18093937, PMID:18250201 Sources: GOC:dph, GOC:jl, GOC:mah Also known as: lipid particle organization and biogenesis, adiposome organization, lipid body organization, lipid particle organisation, lipid particle organization Relationships: is_a organelle organization [GO:0006996] Definition: A process that is carried out at the cellular level which results in the assembly, arrangement of constituent parts, or disassembly of a lipid particle. Subtypes: lipid droplet formation [GO:0140042], GO:0160077, lipid droplet disassembly [GO:1905691]